{
  "gene": "UniProtKB:Q9BU64",
  "term_label": "Unknown biological process",
  "gene_symbol": "CENPO",
  "term_id": "UNKNOWN:0002",
  "gene_name": "Centromere protein O"
}